{
  "gene": "UniProtKB:Q5TCZ1",
  "term_id": "GO:0042554",
  "gene_symbol": "SH3PXD2A",
  "gene_name": "SH3 and PX domain-containing protein 2A",
  "term_label": "superoxide anion generation"
}